{
  "gene_name": "ETS domain-containing protein Elk-4",
  "term_id": "GO:0005634",
  "gene": "UniProtKB:P28324",
  "term_label": "nucleus",
  "gene_symbol": "ELK4"
}